{
  "gene_symbol": "STYXL1",
  "gene_name": "Serine_threonine_tyrosine-interacting-like protein 1",
  "term_id": "GO:0005739",
  "gene": "UniProtKB:Q9Y6J8",
  "term_label": "mitochondrion"
}